{
  "gene": "UniProtKB:A0A1B0GWI6",
  "term_id": "UNKNOWN:0001",
  "gene_symbol": "LOC101059915",
  "term_label": "Unknown molecular function",
  "gene_name": "Uncharacterized protein"
}